1,2-rhamnosyltransferase activity [GO:0102949] (molecular function) References: PMID:15220389 Sources: GOC:pz Relationships: is a type of hexosyltransferase activity [GO:0016758] Definition: Catalysis of the reaction: isoorientin + an L-rhamonsylated rhamnosyl acceptor = isoorientin 2'-O-rhamnoside + a non rhamnosylated rhamnosyl acceptor.